{
  "gene_symbol": "TEX47",
  "gene_name": "Testis-expressed protein 47",
  "term_id": "UNKNOWN:0001",
  "gene": "UniProtKB:Q8TBZ9",
  "term_label": "Unknown molecular function"
}